{
  "term_label": "mitochondrial large ribosomal subunit",
  "term_id": "GO:0005762",
  "gene_name": "Large ribosomal subunit protein uL1m",
  "gene": "UniProtKB:Q9BYD6",
  "gene_symbol": "MRPL1"
}